{
  "term_label": "mitotic spindle",
  "gene": "UniProtKB:Q9ULW0",
  "gene_name": "Targeting protein for Xklp2",
  "gene_symbol": "TPX2",
  "term_id": "GO:0072686"
}